{
  "gene_symbol": "STAT1",
  "gene_name": "Signal transducer and activator of transcription 1-alpha_beta",
  "gene": "UniProtKB:P42224",
  "term_label": "type I interferon-mediated signaling pathway",
  "term_id": "GO:0060337"
}